{
  "gene_symbol": "POC1B",
  "term_id": "UNKNOWN:0001",
  "term_label": "Unknown molecular function",
  "gene_name": "POC1 centriolar protein homolog B",
  "gene": "UniProtKB:Q8TC44"
}